{
  "gene_symbol": "PHYHIPL",
  "term_label": "cytoplasm",
  "gene": "UniProtKB:Q96FC7",
  "gene_name": "Phytanoyl-CoA hydroxylase-interacting protein-like",
  "term_id": "GO:0005737"
}